{
  "term_id": "GO:0000981",
  "term_label": "DNA-binding transcription factor activity, RNA polymerase II-specific",
  "gene": "UniProtKB:P17947",
  "gene_symbol": "SPI1",
  "gene_name": "Transcription factor PU.1"
}